{
  "term_id": "UNKNOWN:0001",
  "term_label": "Unknown molecular function",
  "gene_symbol": "SNTG1",
  "gene_name": "Gamma-1-syntrophin",
  "gene": "UniProtKB:Q9NSN8"
}